{
  "term_id": "GO:0005125",
  "gene_symbol": "IFNA1",
  "gene_name": "Interferon alpha-1_13",
  "term_label": "cytokine activity",
  "gene": "UniProtKB:P01562"
}